{
  "gene": "UniProtKB:Q14289",
  "term_label": "regulation of cell adhesion",
  "term_id": "GO:0030155",
  "gene_name": "Protein-tyrosine kinase 2-beta",
  "gene_symbol": "PTK2B"
}